{
  "term_label": "clathrin binding",
  "term_id": "GO:0030276",
  "gene_symbol": "EPN1",
  "gene_name": "Epsin-1",
  "gene": "UniProtKB:Q9Y6I3"
}